{
  "term_label": "endosomal transport",
  "term_id": "GO:0016197",
  "gene_name": "Vacuolar protein sorting-associated protein 4A",
  "gene_symbol": "VPS4A",
  "gene": "UniProtKB:Q9UN37"
}